{
  "gene_name": "Protein FAM177B",
  "gene": "UniProtKB:A6PVY3",
  "term_id": "UNKNOWN:0003",
  "gene_symbol": "FAM177B",
  "term_label": "Unknown cellular component"
}